{
  "gene_symbol": "C1orf54",
  "term_id": "UNKNOWN:0003",
  "gene_name": "Uncharacterized protein C1orf54",
  "gene": "UniProtKB:Q8WWF1",
  "term_label": "Unknown cellular component"
}